{
  "gene_symbol": "C2orf81",
  "gene": "UniProtKB:A6NN90",
  "term_id": "UNKNOWN:0003",
  "gene_name": "Uncharacterized protein C2orf81",
  "term_label": "Unknown cellular component"
}